negative regulation of molecular function [GO:0044092] (BP) Relationships: is a type of regulation of molecular function [GO:0065009]; negatively regulates molecular_function [GO:0003674] Definition: Any process that stops or reduces the rate or extent of a molecular function, an elemental biological activity occurring at the molecular level, such as catalysis or binding. Sources: GO:jl Subtypes: negative regulation of transporter activity [GO:0032410], negative regulation of ATP-dependent activity [GO:0032780], GO:0043086, negative regulation of DNA-binding transcription factor activity [GO:0043433], negative regulation of binding [GO:0051100], negative regulation of guanyl-nucleotide exchange factor activity [GO:1905098], negative regulation of signaling receptor activity [GO:2000272]